{
  "gene_symbol": "KLC3",
  "gene": "UniProtKB:Q6P597",
  "term_label": "kinesin binding",
  "term_id": "GO:0019894",
  "gene_name": "Kinesin light chain 3"
}